positive regulation of lipopolysaccharide-mediated signaling pathway [GO:0031666] (biological process) Definition: Any process that activates or increases the frequency, rate or extent of signaling in response to detection of lipopolysaccharide. Sources: GOC:mah Relationships: is a type of positive regulation of response to biotic stimulus [GO:0002833]; is a type of GO:0009967; is a type of regulation of lipopolysaccharide-mediated signaling pathway [GO:0031664]; is a type of positive regulation of response to external stimulus [GO:0032103]; positively regulates lipopolysaccharide-mediated signaling pathway [GO:0031663] Also known as: positive regulation of LPS-mediated signaling pathway, positive regulation of lipopolysaccharide-mediated signalling pathway, up regulation of lipopolysaccharide-mediated signaling pathway, up-regulation of lipopolysaccharide-mediated signaling pathway, upregulation of lipopolysaccharide-mediated signaling pathway, activation of lipopolysaccharide-mediated signaling pathway, stimulation of lipopolysaccharide-mediated signaling pathway